regulation of metanephric cap mesenchymal cell proliferation [GO:0090095] (biological process) Sources: GOC:dph, GOC:tb, GOC:yaf Subtypes: positive regulation of metanephric cap mesenchymal cell proliferation [GO:0090096] Definition: Any process that modulates the frequency, rate, or extent of metanephric cap mesenchymal cell proliferation. Metanephric cap mesenchymal cell proliferation is the multiplication or reproduction of metanephric cap mesenchymal cells, resulting in the expansion of the cell population. A metanephric cap mesenchymal cell is a mesenchymal cell that has condensed with other mesenchymal cells surrounding the ureteric bud tip. Relationships: is a type of regulation of mesenchymal cell proliferation [GO:0010464]; is a type of regulation of cell proliferation involved in kidney development [GO:1901722]; regulates GO:0090094